regulation of intracellular mRNA localization [GO:1904580] (biological process) Also known as: regulation of establishment and maintenance of intracellular RNA localization, regulation of intracellular mRNA localisation, regulation of mRNA localization, intracellular, regulation of intracellular mRNA positioning, regulation of mRNA positioning, intracellular Subtypes: regulation of pole plasm oskar mRNA localization [GO:0007317], regulation of bicoid mRNA localization [GO:0008359], GO:1904581, GO:1904582 Definition: Any process that modulates the frequency, rate or extent of intracellular mRNA localization. Relationships: is a type of regulation of localization [GO:0032879]; regulates GO:0008298 References: PMID:21471000 Sources: GOC:TermGenie, GO_REF:0000058